multiple synapse bouton, contacting single dendrite [GO:0150087] (cellular component) Definition: A single axon terminal bouton making contact onto two or more dendritic spines protruding from the same dendrite. Also known as: MSB1, type 1 multi-synapse bouton, type 1 multi-synaptic bouton, type 1 multiple spine synapse bouton, type 1 multiple-synapse bouton, type 1 multisynapse bouton, type 1 multisynaptic bouton Relationships: is a type of multiple synapse bouton [GO:0150086] References: PMID:10586883, PMID:11248111, PMID:22028887, PMID:24487234 Sources: GOC:aruk, GOC:bc